{
  "gene": "UniProtKB:Q6NZY7",
  "gene_name": "Cdc42 effector protein 5",
  "term_label": "positive regulation of actin filament polymerization",
  "gene_symbol": "CDC42EP5",
  "term_id": "GO:0030838"
}